{
  "term_id": "GO:0010507",
  "gene_name": "Ras-related GTP-binding protein C",
  "term_label": "negative regulation of autophagy",
  "gene_symbol": "RRAGC",
  "gene": "UniProtKB:Q9HB90"
}